regulation of filamentous growth of a population of unicellular organisms in response to chemical stimulus [GO:1900437] (biological process) Definition: Any process that modulates the frequency, rate or extent of filamentous growth of a population of unicellular organisms in response to chemical stimulus. Sources: GOC:TermGenie, GOC:di Relationships: is a type of regulation of response to stimulus [GO:0048583]; is_a regulation of filamentous growth of a population of unicellular organisms [GO:1900428]; regulates filamentous growth of a population of unicellular organisms in response to chemical stimulus [GO:0036171] Subtypes: negative regulation of filamentous growth of a population of unicellular organisms in response to chemical stimulus [GO:1900438], positive regulation of filamentous growth of a population of unicellular organisms in response to chemical stimulus [GO:1900439]